tripeptide transmembrane transporter activity [GO:0042937] (molecular function) Relationships: is a type of oligopeptide transmembrane transporter activity [GO:0035673]; is part of GO:0042939 Sources: GOC:jl Subtypes: glutathione transmembrane transporter activity [GO:0034634] Also known as: tripeptide transporter activity Definition: Enables the transfer of a tripeptide, a compound containing three amino acids linked together by peptide bonds, from one side of a membrane to the other.